{
  "gene_name": "Filamin-binding LIM protein 1",
  "term_label": "stress fiber",
  "gene_symbol": "FBLIM1",
  "term_id": "GO:0001725",
  "gene": "UniProtKB:Q8WUP2"
}